{
  "gene": "UniProtKB:P14416",
  "gene_symbol": "DRD2",
  "term_label": "negative regulation of synaptic transmission, glutamatergic",
  "term_id": "GO:0051967",
  "gene_name": "D(2) dopamine receptor"
}